{
  "term_id": "GO:0031053",
  "gene": "UniProtKB:Q8WYQ5",
  "gene_symbol": "DGCR8",
  "term_label": "primary miRNA processing",
  "gene_name": "Microprocessor complex subunit DGCR8"
}